{
  "gene_name": "C-type lectin domain family 2 member A",
  "gene": "UniProtKB:Q6UVW9",
  "gene_symbol": "CLEC2A",
  "term_id": "GO:0050852",
  "term_label": "T cell receptor signaling pathway"
}